laminin-8 complex [GO:0043257] (cellular component) Relationships: is a type of GO:0043256 References: PMID:10842354 Sources: GOC:jl Definition: A laminin complex composed of alpha4, beta1 and gamma1 polypeptide chains. Also known as: laminin-411 complex